{
  "term_label": "semaphorin receptor activity",
  "gene_symbol": "PLXNB2",
  "gene_name": "Plexin-B2",
  "term_id": "GO:0017154",
  "gene": "UniProtKB:O15031"
}